{
  "gene_name": "BTB_POZ domain-containing protein KCTD20",
  "gene": "UniProtKB:Q7Z5Y7",
  "term_label": "Unknown molecular function",
  "gene_symbol": "KCTD20",
  "term_id": "UNKNOWN:0001"
}